negative regulation of myofibroblast differentiation [GO:1904761] (BP) Definition: Any process that stops, prevents or reduces the frequency, rate or extent of myofibroblast differentiation. Also known as: down regulation of myofibroblast cell differentiation, down regulation of myofibroblast differentiation, down-regulation of myofibroblast cell differentiation, down-regulation of myofibroblast differentiation, downregulation of myofibroblast cell differentiation, downregulation of myofibroblast differentiation, negative regulation of myofibroblast cell differentiation, inhibition of myofibroblast cell differentiation, inhibition of myofibroblast differentiation References: PMID:20533548 Sources: GOC:BHF, GOC:BHF_miRNA, GOC:TermGenie, GOC:rph, GO_REF:0000058 Relationships: is a type of negative regulation of cell differentiation [GO:0045596]; is a type of regulation of myofibroblast differentiation [GO:1904760]; negatively regulates myofibroblast differentiation [GO:0036446]